laminated body [GO:1990011] (CC) Also known as: laminated inclusion body Sources: ISBN:0195065719, NIF_Subcellular:sao506721981 Subtypes: complex laminated body [GO:1990012] Relationships: is_a inclusion body [GO:0016234] Definition: Inclusion body characterized by regularly spaced sheets of tubules arranged in a whorl pattern resembling a fingerprint. Laminated bodies have been observed in neurons of the lateral geniculate nucleus.